{
  "term_label": "Unknown biological process",
  "gene_symbol": "FUT2",
  "gene": "UniProtKB:Q10981",
  "term_id": "UNKNOWN:0002",
  "gene_name": "Galactoside alpha-(1,2)-fucosyltransferase 2"
}